{
  "gene": "UniProtKB:A0A8V8TII8",
  "term_label": "Unknown cellular component",
  "gene_name": "Uncharacterized protein",
  "term_id": "UNKNOWN:0003",
  "gene_symbol": "A0A8V8TII8"
}